plastid acetyl-CoA carboxylase complex [GO:0032282] (cellular component) Definition: An acetyl-CoA carboxylase complex located in the stroma of a plastid. Relationships: is a type of GO:0009317; is part of plastid stroma [GO:0009532] Sources: GOC:mah Also known as: plastid ACCase complex